{
  "gene_name": "Bifunctional peptidase and arginyl-hydroxylase JMJD5",
  "term_id": "GO:0005634",
  "gene_symbol": "KDM8",
  "gene": "UniProtKB:Q8N371",
  "term_label": "nucleus"
}